{
  "gene_name": "Na(+)_H(+) exchange regulatory cofactor NHE-RF4",
  "term_id": "GO:0043495",
  "gene_symbol": "NHERF4",
  "gene": "UniProtKB:Q86UT5",
  "term_label": "protein-membrane adaptor activity"
}